retinal rod cell fate commitment [GO:0060223] (BP) Definition: The process in which the developmental fate of a cell becomes restricted such that it will develop into a retinal rod cell. A retinal rod cell is one of the two photoreceptor subtypes in a camera-type eye. Sources: GOC:dph Relationships: is a type of camera-type eye photoreceptor cell fate commitment [GO:0060220]; is part of retinal rod cell differentiation [GO:0060221] Regulation: regulated by regulation of retinal rod cell fate commitment [GO:0060224]; RO_0002213 by positive regulation of retinal rod cell fate commitment [GO:0060225]